{
  "gene_name": "Putative golgin subfamily A member 6-like protein 19",
  "term_label": "Unknown molecular function",
  "term_id": "UNKNOWN:0001",
  "gene_symbol": "GOLGA6L19",
  "gene": "UniProtKB:H0YKK7"
}